{
  "gene_name": "Guanine deaminase",
  "term_id": "GO:0046098",
  "gene_symbol": "GDA",
  "term_label": "guanine metabolic process",
  "gene": "UniProtKB:Q9Y2T3"
}